eoxin E4 synthase activity [GO:0097263] (molecular function) Relationships: is a type of GO:0008238 References: PMID:18184802, PMID:18647347 Sources: GOC:mw Definition: Catalysis of the reaction: eoxin D4 + H20 = eoxin E4 + glycine.